{
  "gene": "UniProtKB:Q8TF47",
  "term_id": "GO:0000977",
  "gene_symbol": "ZFP90",
  "gene_name": "Zinc finger protein 90 homolog",
  "term_label": "RNA polymerase II transcription regulatory region sequence-specific DNA binding"
}